{
  "term_id": "GO:0035338",
  "gene": "UniProtKB:Q9ULC5",
  "gene_symbol": "ACSL5",
  "gene_name": "Long-chain-fatty-acid--CoA ligase 5",
  "term_label": "long-chain fatty-acyl-CoA biosynthetic process"
}